{
  "gene_name": "Rho guanine nucleotide exchange factor 7",
  "term_id": "GO:0005737",
  "gene": "UniProtKB:Q14155",
  "gene_symbol": "ARHGEF7",
  "term_label": "cytoplasm"
}